cardiogenic plate morphogenesis [GO:0003142] (biological process) Also known as: cardiac crescent morphogenesis Relationships: is a type of anatomical structure morphogenesis [GO:0009653]; is part of heart morphogenesis [GO:0003007] Definition: The process in which the anatomical structures of the cardiogenic plate are generated and organized. The cardiogenic plate is the first recognizable structure derived from the heart field. Sources: GOC:mtg_heart